negative regulation of skeletal muscle contraction by regulation of release of sequestered calcium ion [GO:0014811] (biological process) Definition: Any process that stops, prevents, or reduces the frequency, rate or extent of skeletal muscle contraction via the regulation of the release of sequestered calcium ion by sarcoplasmic reticulum into cytosol. The sarcoplasmic reticulum is the endoplasmic reticulum of striated muscle, specialised for the sequestration of calcium ions that are released upon receipt of a signal relayed by the T tubules from the neuromuscular junction. Sources: GOC:mtg_muscle Relationships: is a type of GO:0014809; is a type of negative regulation of striated muscle contraction [GO:0045988]